{
  "term_label": "centriole replication",
  "term_id": "GO:0007099",
  "gene_name": "Centrosomal protein of 72 kDa",
  "gene_symbol": "CEP72",
  "gene": "UniProtKB:Q9P209"
}